{
  "term_label": "heat shock protein binding",
  "gene": "UniProtKB:P11142",
  "term_id": "GO:0031072",
  "gene_symbol": "HSPA8",
  "gene_name": "Heat shock cognate 71 kDa protein"
}